{
  "gene_symbol": "HINT3",
  "term_id": "UNKNOWN:0001",
  "gene": "UniProtKB:Q9NQE9",
  "term_label": "Unknown molecular function",
  "gene_name": "Adenosine 5'-monophosphoramidase HINT3"
}